{
  "term_id": "GO:0022857",
  "gene": "UniProtKB:Q9BS91",
  "gene_symbol": "SLC35A5",
  "gene_name": "Probable UDP-sugar transporter protein SLC35A5",
  "term_label": "transmembrane transporter activity"
}